{
  "gene": "UniProtKB:Q5TBB1",
  "term_label": "Unknown molecular function",
  "gene_symbol": "RNASEH2B",
  "term_id": "UNKNOWN:0001",
  "gene_name": "Ribonuclease H2 subunit B"
}